negative regulation of production of molecular mediator of immune response [GO:0002701] (biological process) Also known as: down regulation of production of molecular mediator of immune response, down-regulation of production of molecular mediator of immune response, downregulation of production of molecular mediator of immune response, inhibition of production of molecular mediator of immune response Relationships: is a type of GO:0002698; is_a regulation of production of molecular mediator of immune response [GO:0002700]; is a type of negative regulation of gene expression [GO:0010629]; negatively regulates GO:0002440 Sources: GOC:add Subtypes: negative regulation of immunoglobulin production [GO:0002638], negative regulation of cytokine production involved in immune response [GO:0002719], GO:0002785, GO:0071662, negative regulation of granzyme A production [GO:2000512] Definition: Any process that stops, prevents, or reduces the frequency, rate, or extent of the production of molecular mediator of immune response.